photosystem II oxygen evolving complex [GO:0009654] (CC) Also known as: OEC (PSII) complex, oxygen evolving complex Sources: GOC:cjm, InterPro:IPR002683 Relationships: is_a membrane protein complex [GO:0098796]; is_a oxidoreductase complex [GO:1990204]; is part of photosystem II [GO:0009523]; is part of thylakoid membrane [GO:0042651] Definition: A complex, composed of a cluster of manganese, calcium and chloride ions bound to extrinsic proteins, that catalyzes the splitting of water to O2 and 4 H+. In cyanobacteria there are five extrinsic proteins in OEC (PsbO, PsbP-like, PsbQ-like, PsbU and PsbV), while in plants there are only three (PsbO, PsbP and PsbQ).